{
  "gene_name": "Golgin subfamily A member 6B",
  "gene_symbol": "GOLGA6B",
  "gene": "UniProtKB:A6NDN3",
  "term_label": "cis-Golgi network",
  "term_id": "GO:0005801"
}